{
  "gene_name": "PAS domain-containing serine_threonine-protein kinase",
  "gene": "UniProtKB:Q96RG2",
  "term_label": "negative regulation of glycogen biosynthetic process",
  "term_id": "GO:0045719",
  "gene_symbol": "PASK"
}